{
  "gene_symbol": "GNAZ",
  "gene_name": "Guanine nucleotide-binding protein G(z) subunit alpha",
  "gene": "UniProtKB:P19086",
  "term_id": "GO:0003924",
  "term_label": "GTPase activity"
}